{
  "term_label": "extracellular region",
  "gene_symbol": "CRIPTO3",
  "gene": "UniProtKB:P51864",
  "gene_name": "Putative teratocarcinoma-derived growth factor 3",
  "term_id": "GO:0005576"
}